{
  "gene_symbol": "NSRP1",
  "term_id": "UNKNOWN:0003",
  "gene": "UniProtKB:Q9H0G5",
  "gene_name": "Nuclear speckle splicing regulatory protein 1",
  "term_label": "Unknown cellular component"
}